{
  "term_label": "mitotic G2 DNA damage checkpoint signaling",
  "gene": "UniProtKB:P06493",
  "gene_symbol": "CDK1",
  "gene_name": "Cyclin-dependent kinase 1",
  "term_id": "GO:0007095"
}